{
  "gene_name": "Coiled-coil domain-containing protein 137",
  "term_id": "UNKNOWN:0001",
  "gene_symbol": "CCDC137",
  "gene": "UniProtKB:Q6PK04",
  "term_label": "Unknown molecular function"
}